{
  "gene_name": "Nucleolar protein 56",
  "term_id": "GO:0031428",
  "gene_symbol": "NOP56",
  "term_label": "box C/D methylation guide snoRNP complex",
  "gene": "UniProtKB:O00567"
}